{
  "gene": "UniProtKB:A0A183",
  "term_id": "UNKNOWN:0001",
  "gene_name": "Late cornified envelope protein 6A",
  "term_label": "Unknown molecular function",
  "gene_symbol": "LCE6A"
}